{
  "gene": "UniProtKB:Q9ULE6",
  "term_label": "cytoplasm",
  "gene_symbol": "PALD1",
  "term_id": "GO:0005737",
  "gene_name": "Paladin"
}